{
  "gene_symbol": "ZNF264",
  "gene": "UniProtKB:O43296",
  "term_id": "GO:0005634",
  "term_label": "nucleus",
  "gene_name": "Zinc finger protein 264"
}